{
  "term_id": "UNKNOWN:0003",
  "term_label": "Unknown cellular component",
  "gene_name": "Beta-defensin 134",
  "gene_symbol": "DEFB134",
  "gene": "UniProtKB:Q4QY38"
}